pollen exine formation [GO:0010584] (biological process) Sources: GOC:dhl Definition: The formation of the pollen exine. The reticulate pollen wall pattern consists of two layers, exine and intine. Relationships: is a type of pollen wall assembly [GO:0010208]